lamina terminalis formation [GO:0021996] (biological process) Relationships: is_a anatomical structure formation involved in morphogenesis [GO:0048646]; is part of anterior neuropore closure [GO:0021506] Definition: The process in which the anterior-most portion of the neural axis is formed by closure of the anterior neuropore. Sources: GOC:cls, GOC:dgh, GOC:dph, GOC:jid, GO_REF:0000021